{
  "gene_name": "Cystatin-SA",
  "term_label": "cytoplasm",
  "gene": "UniProtKB:P09228",
  "term_id": "GO:0005737",
  "gene_symbol": "CST2"
}